positive regulation of phenazine biosynthetic process [GO:1900982] (BP) Also known as: up regulation of phenazine biosynthetic process, up-regulation of phenazine biosynthetic process, upregulation of phenazine biosynthetic process, activation of phenazine biosynthetic process, activation of acridizine biosynthesis, activation of acridizine biosynthetic process, activation of azophenylene biosynthesis, activation of azophenylene biosynthetic process, activation of dibenzo-p-diazine biosynthesis, activation of dibenzo-p-diazine biosynthetic process, activation of dibenzopyrazine biosynthesis, activation of dibenzopyrazine biosynthetic process, positive regulation of acridizine biosynthesis, positive regulation of acridizine biosynthetic process, positive regulation of azophenylene biosynthesis, positive regulation of azophenylene biosynthetic process, positive regulation of dibenzo-p-diazine biosynthesis, positive regulation of dibenzo-p-diazine biosynthetic process, positive regulation of dibenzopyrazine biosynthesis, positive regulation of dibenzopyrazine biosynthetic process, up regulation of acridizine biosynthesis, up regulation of acridizine biosynthetic process, up regulation of azophenylene biosynthesis, up regulation of azophenylene biosynthetic process, up regulation of dibenzo-p-diazine biosynthesis, up regulation of dibenzo-p-diazine biosynthetic process, up regulation of dibenzopyrazine biosynthesis, up regulation of dibenzopyrazine biosynthetic process, up-regulation of acridizine biosynthesis, up-regulation of acridizine biosynthetic process, up-regulation of azophenylene biosynthesis, up-regulation of azophenylene biosynthetic process, up-regulation of dibenzo-p-diazine biosynthesis, up-regulation of dibenzo-p-diazine biosynthetic process, up-regulation of dibenzopyrazine biosynthesis, up-regulation of dibenzopyrazine biosynthetic process, upregulation of acridizine biosynthesis, upregulation of acridizine biosynthetic process, upregulation of azophenylene biosynthesis, upregulation of azophenylene biosynthetic process, upregulation of dibenzo-p-diazine biosynthesis, upregulation of dibenzo-p-diazine biosynthetic process, upregulation of dibenzopyrazine biosynthesis, upregulation of dibenzopyrazine biosynthetic process Relationships: is a type of positive regulation of biosynthetic process [GO:0009891]; is a type of regulation of phenazine biosynthetic process [GO:1900980]; positively regulates phenazine biosynthetic process [GO:0002047] Sources: GOC:TermGenie, GOC:mengo_curators Definition: Any process that activates or increases the frequency, rate or extent of phenazine biosynthetic process.